{
  "gene_name": "6-phosphofructo-2-kinase_fructose-2,6-bisphosphatase 3",
  "term_label": "6-phosphofructo-2-kinase activity",
  "gene": "UniProtKB:Q16875",
  "gene_symbol": "PFKFB3",
  "term_id": "GO:0003873"
}